{
  "gene_name": "Mothers against decapentaplegic homolog 9",
  "gene_symbol": "SMAD9",
  "gene": "UniProtKB:O15198",
  "term_label": "I-SMAD binding",
  "term_id": "GO:0070411"
}